nucleosome [GO:0000786] (cellular component) Definition: A complex comprised of DNA wound around a multisubunit core and associated proteins, which forms the primary packing unit of DNA into higher order structures. Sources: GOC:elh Also known as: cytoplasmic nucleosome, nuclear nucleosome Relationships: is a type of GO:0032993; is part of chromatin [GO:0000785] Subtypes: CENP-A containing nucleosome [GO:0043505], histone H3-containing nucleosome [GO:0140573]